positive regulation of toll-like receptor 12 signaling pathway [GO:0034177] (biological process) Also known as: positive regulation of TLR12 signaling pathway, positive regulation of toll-like receptor 12 signalling pathway Relationships: is a type of regulation of toll-like receptor 12 signaling pathway [GO:0034175]; is a type of positive regulation of pattern recognition receptor signaling pathway [GO:0062208]; is a type of positive regulation of intracellular signal transduction [GO:1902533]; positively regulates toll-like receptor 12 signaling pathway [GO:0034174] Definition: Any process that activates or increases the frequency, rate, or extent of toll-like receptor 12 signaling pathway. References: PMID:16551253, PMID:17328678 Sources: GOC:add